{
  "gene": "UniProtKB:Q96CW6",
  "term_label": "Unknown molecular function",
  "term_id": "UNKNOWN:0001",
  "gene_symbol": "SLC7A6OS",
  "gene_name": "Probable RNA polymerase II nuclear localization protein SLC7A6OS"
}